{
  "term_id": "GO:0160077",
  "gene_symbol": "CIDEA",
  "gene_name": "Lipid transferase CIDEA",
  "gene": "UniProtKB:O60543",
  "term_label": "lipid droplet fusion"
}